negative regulation of cell maturation [GO:1903430] (biological process) Subtypes: negative regulation of neuron maturation [GO:0014043], negative regulation of erythrocyte enucleation [GO:0061932], negative regulation of oocyte maturation [GO:1900194], negative regulation of sperm capacitation [GO:1902491], negative regulation of root hair elongation [GO:1902891] References: PMID:17459944 Sources: GOC:TermGenie, GO_REF:0000058 Also known as: down regulation of cell maturation, down-regulation of cell maturation, downregulation of cell maturation, inhibition of cell maturation, down regulation of functional differentiation, down-regulation of functional differentiation, downregulation of functional differentiation, inhibition of functional differentiation, negative regulation of functional differentiation Definition: Any process that stops, prevents or reduces the frequency, rate or extent of cell maturation. Relationships: is a type of GO:0010721; is a type of regulation of cell maturation [GO:1903429]; negatively regulates cell maturation [GO:0048469]